deoxyribonucleoside triphosphate metabolic process [GO:0009200] (biological process) Sources: GOC:go_curators, ISBN:0198506732 Subtypes: deoxyribonucleoside triphosphate biosynthetic process [GO:0009202], deoxyribonucleoside triphosphate catabolic process [GO:0009204], purine deoxyribonucleoside triphosphate metabolic process [GO:0009215] Relationships: is a type of GO:0009141 Also known as: deoxyribonucleoside triphosphate metabolism Definition: The chemical reactions and pathways involving a deoxyribonucleoside triphosphate, a compound consisting of a nucleobase linked to a deoxyribose sugar esterified with triphosphate on the sugar.